{
  "gene_name": "Cyclin-dependent kinase 2",
  "term_id": "GO:0007165",
  "gene_symbol": "CDK2",
  "term_label": "signal transduction",
  "gene": "UniProtKB:P24941"
}